cytochrome c metabolic process [GO:1903606] (biological process) Subtypes: GO:1903607 Relationships: is a type of cytochrome metabolic process [GO:1903604] References: PMID:19721088 Sources: GOC:TermGenie, GOC:dph, GO_REF:0000068 Also known as: cytochrome c metabolism Definition: The chemical reactions and pathways involving cytochrome c.